{
  "gene_name": "Ganglioside-induced differentiation-associated protein 2",
  "term_id": "UNKNOWN:0003",
  "gene_symbol": "GDAP2",
  "gene": "UniProtKB:Q9NXN4",
  "term_label": "Unknown cellular component"
}